plant-type sporogenesis [GO:0048236] (biological process) Definition: The formation of plant spores derived from the products of meiosis. The spore gives rise to gametophytes. Sources: GOC:tb Also known as: plant spore formation Relationships: is a type of GO:0034293; is a type of cellular developmental process [GO:0048869]; is a type of GO:0051321; is a type of meiotic cell cycle process [GO:1903046] Subtypes: megasporogenesis [GO:0009554], microsporogenesis [GO:0009556]